MAP-kinase scaffold activity [GO:0005078] (molecular function) Also known as: MAP-kinase scaffold protein activity References: PMID:12511654, PMID:15213240, PMID:9405336 Relationships: is a type of signaling adaptor activity [GO:0035591]; BFO_0000050 GO:0000165; has part mitogen-activated protein kinase binding [GO:0051019] Definition: The binding activity of a molecule that functions as a physical support for the assembly of a multiprotein mitogen-activated protein kinase (MAPK) complex. Binds multiple kinases of the MAPKKK cascade, and also upstream signaling proteins, permitting those molecules to function in a coordinated way. Bringing together multiple enzymes and their substrates enables the signal to be transduced quickly and efficiently.